{
  "term_label": "intracellular signal transduction",
  "gene_name": "Serine_threonine-protein kinase Nek4",
  "gene": "UniProtKB:P51957",
  "term_id": "GO:0035556",
  "gene_symbol": "NEK4"
}